{
  "term_id": "GO:0005654",
  "term_label": "nucleoplasm",
  "gene_name": "Ribosomal protein S6 kinase beta-1",
  "gene": "UniProtKB:P23443",
  "gene_symbol": "RPS6KB1"
}